{
  "term_id": "GO:0000978",
  "term_label": "RNA polymerase II cis-regulatory region sequence-specific DNA binding",
  "gene": "UniProtKB:P48378",
  "gene_symbol": "RFX2",
  "gene_name": "DNA-binding protein RFX2"
}